negative regulation of interleukin-23 production [GO:0032707] (biological process) Sources: GOC:mah Also known as: down regulation of interleukin-23 production, down-regulation of interleukin-23 production, downregulation of interleukin-23 production, negative regulation of IL-23 production, inhibition of interleukin-23 production, negative regulation of interleukin-23 biosynthetic process Relationships: is a type of GO:0001818; is a type of regulation of interleukin-23 production [GO:0032667]; negatively regulates interleukin-23 production [GO:0032627] Definition: Any process that stops, prevents, or reduces the frequency, rate, or extent of interleukin-23 production.